{
  "gene_name": "G-protein coupled receptor 143",
  "gene_symbol": "GPR143",
  "term_id": "GO:0035240",
  "term_label": "dopamine binding",
  "gene": "UniProtKB:P51810"
}